mesendoderm development [GO:0048382] (biological process) Definition: The process whose specific outcome is the progression of the mesendoderm over time, from its formation to the mature structure. In animal embryos, mesendoderm development gives rise to both mesoderm and endoderm tissues. Sources: GOC:jid Relationships: is a type of GO:0048856; is part of endoderm development [GO:0007492]; is part of mesoderm development [GO:0007498]